histone H2AK129 ubiquitin ligase activity [GO:0140864] (MF) Also known as: histone H2A-K129 ubiquitin ligase activity, histone ubiquitin ligase activity (H2A-K129 specific) References: PMID:28624371 Relationships: is a type of histone H2A ubiquitin ligase activity [GO:0141053] Definition: Catalysis of the transfer of a ubiquitin molecule to histone 2A at the lysine-129 residue. Note: Note that the residue position corresponds to the canonical human H2A2A histone (UniProtKB:Q6FI13); this residue is only present in vertebrates. Residue 1 is the first residue following removal of the initiating Methionine (Met). Note that each histone is encoded by multiple genes, and sequences may vary across different genes within an organism.